{
  "gene": "UniProtKB:Q8IWA4",
  "term_id": "GO:0003924",
  "gene_symbol": "MFN1",
  "gene_name": "Mitofusin-1",
  "term_label": "GTPase activity"
}